{
  "term_label": "Unknown cellular component",
  "term_id": "UNKNOWN:0003",
  "gene_name": "Mitochondrial antiviral-signaling protein",
  "gene_symbol": "MAVS",
  "gene": "UniProtKB:Q7Z434"
}